{
  "gene_symbol": "ANGPTL6",
  "term_id": "UNKNOWN:0002",
  "gene_name": "Angiopoietin-related protein 6",
  "gene": "UniProtKB:Q8NI99",
  "term_label": "Unknown biological process"
}